{
  "gene": "UniProtKB:P22459",
  "gene_symbol": "KCNA4",
  "term_label": "delayed rectifier potassium channel activity",
  "gene_name": "Potassium voltage-gated channel subfamily A member 4",
  "term_id": "GO:0005251"
}